{
  "gene_name": "Cilia- and flagella-associated protein 46",
  "gene_symbol": "CFAP46",
  "term_id": "UNKNOWN:0001",
  "term_label": "Unknown molecular function",
  "gene": "UniProtKB:Q8IYW2"
}